{
  "gene_name": "Destrin",
  "term_id": "GO:0030043",
  "gene": "UniProtKB:P60981",
  "gene_symbol": "DSTN",
  "term_label": "actin filament fragmentation"
}